{
  "term_label": "Unknown cellular component",
  "gene_symbol": "DGCR6",
  "term_id": "UNKNOWN:0003",
  "gene": "UniProtKB:Q14129",
  "gene_name": "Protein DGCR6"
}